{
  "gene": "UniProtKB:Q6NVY1",
  "gene_symbol": "HIBCH",
  "gene_name": "3-hydroxyisobutyryl-CoA hydrolase, mitochondrial",
  "term_label": "mitochondrion",
  "term_id": "GO:0005739"
}